{
  "gene": "UniProtKB:Q9BTZ2",
  "term_id": "GO:0005777",
  "gene_symbol": "DHRS4",
  "term_label": "peroxisome",
  "gene_name": "Dehydrogenase_reductase SDR family member 4"
}